{
  "term_label": "Unknown molecular function",
  "gene_symbol": "TWSG1",
  "term_id": "UNKNOWN:0001",
  "gene": "UniProtKB:Q9GZX9",
  "gene_name": "Twisted gastrulation protein homolog 1"
}